{
  "gene": "UniProtKB:Q96BF6",
  "gene_symbol": "NACC2",
  "gene_name": "Nucleus accumbens-associated protein 2",
  "term_id": "GO:0006357",
  "term_label": "regulation of transcription by RNA polymerase II"
}